internode region of axon [GO:0033269] (cellular component) Relationships: is a type of GO:0110165; is part of GO:0044304 Also known as: internode Sources: GOC:mah, GOC:mh Definition: An axon part that is located between the nodes of Ranvier and surrounded by compact myelin sheath.